{
  "gene_symbol": "GCLC",
  "term_id": "GO:0017109",
  "gene_name": "Glutamate--cysteine ligase catalytic subunit",
  "term_label": "glutamate-cysteine ligase complex",
  "gene": "UniProtKB:P48506"
}